negative regulation of integrin biosynthetic process [GO:0045720] (biological process) Subtypes: negative regulation of beta 2 integrin biosynthetic process [GO:0045774] Definition: Any process that stops, prevents, or reduces the frequency, rate or extent of the chemical reactions and pathways resulting in the formation of integrins. Relationships: is_a GO:0010558; is a type of regulation of integrin biosynthetic process [GO:0045113]; is a type of GO:0051129; negatively regulates GO:0045112 Also known as: down regulation of integrin biosynthetic process, down-regulation of integrin biosynthetic process, downregulation of integrin biosynthetic process, negative regulation of integrin anabolism, negative regulation of integrin biosynthesis, negative regulation of integrin formation, negative regulation of integrin synthesis, inhibition of integrin biosynthetic process Sources: GOC:go_curators